{
  "term_id": "GO:0061630",
  "gene_symbol": "UBR4",
  "term_label": "ubiquitin protein ligase activity",
  "gene": "UniProtKB:Q5T4S7",
  "gene_name": "E3 ubiquitin-protein ligase UBR4"
}